{
  "term_label": "Unknown molecular function",
  "gene_name": "Mth938 domain-containing protein",
  "gene": "UniProtKB:Q9H7C9",
  "gene_symbol": "AAMDC",
  "term_id": "UNKNOWN:0001"
}